{
  "term_label": "tubulin binding",
  "gene_symbol": "TPPP3",
  "gene_name": "Tubulin polymerization-promoting protein family member 3",
  "term_id": "GO:0015631",
  "gene": "UniProtKB:Q9BW30"
}